{
  "term_id": "GO:0005886",
  "gene": "UniProtKB:Q99679",
  "gene_symbol": "GPR21",
  "gene_name": "Probable G-protein coupled receptor 21",
  "term_label": "plasma membrane"
}